DNA methylation-dependent constitutive heterochromatin formation [GO:0006346] (biological process) Definition: Formation of constitutive heterochromatin by a pathway that includes methylation of genomic DNA such as CpG islands. Sources: GOC:mah Also known as: methylation-dependent chromatin silencing, methylation-dependent heterochromatic silencing, DNA methylation-dependent heterochromatin assembly, DNA methylation-dependent heterochromatin formation Relationships: is a type of GO:0140719 Subtypes: GO:0080188, gene silencing by piRNA-directed DNA methylation [GO:0141176] Regulation: negatively regulated by negative regulation of DNA methylation-dependent heterochromatin formation [GO:0090310]